{
  "term_label": "Unknown cellular component",
  "gene": "UniProtKB:O43451",
  "term_id": "UNKNOWN:0003",
  "gene_symbol": "MGAM",
  "gene_name": "Maltase-glucoamylase"
}